{
  "gene": "UniProtKB:Q13426",
  "gene_name": "DNA repair protein XRCC4",
  "gene_symbol": "XRCC4",
  "term_label": "DNA ligase IV complex",
  "term_id": "GO:0032807"
}